{
  "term_label": "transcription regulator complex",
  "term_id": "GO:0005667",
  "gene": "UniProtKB:Q8IZ40",
  "gene_name": "REST corepressor 2",
  "gene_symbol": "RCOR2"
}